{
  "term_label": "protein tyrosine kinase activity",
  "gene": "UniProtKB:P00519",
  "gene_symbol": "ABL1",
  "term_id": "GO:0004713",
  "gene_name": "Tyrosine-protein kinase ABL1"
}